{
  "gene_name": "Exosome complex component RRP42",
  "gene": "UniProtKB:Q15024",
  "term_label": "cytoplasmic exosome (RNase complex)",
  "gene_symbol": "EXOSC7",
  "term_id": "GO:0000177"
}